{
  "gene_symbol": "SYT11",
  "gene": "UniProtKB:Q9BT88",
  "term_label": "calcium-dependent phospholipid binding",
  "gene_name": "Synaptotagmin-11",
  "term_id": "GO:0005544"
}